venom-mediated vasodilation by activation of bradykinin receptor signaling pathway [GO:0140162] (biological process) Relationships: is a type of venom-mediated perturbation of G protein-coupled receptor signaling pathway [GO:0044513]; is a type of venom-mediated vasodilation [GO:0044551] References: PMID:31370142 Also known as: venom-mediated vasodilation by activation of bradykinin-dependent signaling, venom-mediated vasodilation through activity of bradykinin Definition: A process in which an organism initiates, promotes, or enhances vasodilation via the action of a venom that activates bradykinin-dependent signaling, concomittantly reducing blood pressure in the bitten/stung organism. This can take place via several mechanisms that affect endogenous bradykinin: either increasing its release by kallikrein-like proteases, increasing bradykinin action by potentiation, or inhibiting bradykinin degradation.